microneme lumen [GO:0034494] (cellular component) Sources: GOC:rph Relationships: is a type of intracellular organelle lumen [GO:0070013]; is part of GO:0020009 Definition: The volume enclosed by the microneme membrane.